{
  "gene_symbol": "WDR3",
  "term_label": "maturation of SSU-rRNA",
  "term_id": "GO:0030490",
  "gene_name": "WD repeat-containing protein 3",
  "gene": "UniProtKB:Q9UNX4"
}